{
  "term_label": "oxalate transmembrane transporter activity",
  "gene_symbol": "SLC26A9",
  "gene_name": "Solute carrier family 26 member 9",
  "term_id": "GO:0019531",
  "gene": "UniProtKB:Q7LBE3"
}